{
  "gene": "UniProtKB:P49821",
  "gene_name": "NADH dehydrogenase [ubiquinone] flavoprotein 1, mitochondrial",
  "term_id": "GO:0006120",
  "gene_symbol": "NDUFV1",
  "term_label": "mitochondrial electron transport, NADH to ubiquinone"
}